regulation of chlorophyll metabolic process [GO:0090056] (biological process) Relationships: is a type of GO:1901401; regulates chlorophyll metabolic process [GO:0015994] Sources: GOC:dph, GOC:tb Definition: Any process that modulates the frequency, rate or extent of the chemical reactions and pathways involving chlorophyll. Subtypes: GO:0010271, regulation of chlorophyll biosynthetic process [GO:0010380]